{
  "term_label": "U6 snRNP",
  "gene": "UniProtKB:Q9Y333",
  "gene_symbol": "LSM2",
  "term_id": "GO:0005688",
  "gene_name": "U6 snRNA-associated Sm-like protein LSm2"
}